{
  "gene": "UniProtKB:P55895",
  "term_label": "V(D)J recombination",
  "gene_name": "V(D)J recombination-activating protein 2",
  "gene_symbol": "RAG2",
  "term_id": "GO:0033151"
}